{
  "gene_symbol": "SMAD9",
  "gene_name": "Mothers against decapentaplegic homolog 9",
  "term_label": "BMP signaling pathway",
  "term_id": "GO:0030509",
  "gene": "UniProtKB:O15198"
}